{
  "gene_name": "Nuclear receptor subfamily 1 group D member 2",
  "gene": "UniProtKB:Q14995",
  "term_label": "positive regulation of transcription by RNA polymerase II",
  "term_id": "GO:0045944",
  "gene_symbol": "NR1D2"
}